{
  "gene_name": "FXYD domain-containing ion transport regulator 7",
  "term_label": "sodium channel regulator activity",
  "gene": "UniProtKB:P58549",
  "gene_symbol": "FXYD7",
  "term_id": "GO:0017080"
}